{
  "term_label": "defense response to Gram-positive bacterium",
  "term_id": "GO:0050830",
  "gene_name": "N-acetylmuramoyl-L-alanine amidase",
  "gene_symbol": "PGLYRP2",
  "gene": "UniProtKB:Q96PD5"
}